4-nitrophenol 4-monooxygenase activity [GO:0018632] (molecular function) Definition: Catalysis of the reaction: p-nitrophenol + O2 + NADPH = H2O + NADP+ + nitrite + p-benzoquinone. Sources: RHEA:34327 Relationships: is a type of GO:0016709